(1->6)-beta-D-glucan binding [GO:2001078] (molecular function) Definition: Binding to (1->6)-beta-D-glucan. Relationships: is a type of polysaccharide binding [GO:0030247] Also known as: (1,6)-beta-D-glucan binding, 1,6-beta-D-glucan binding, 1->6-beta-D-glucan binding, beta-(1,6)-D-glucan binding, beta-(1->6)-D-glucan binding, beta-1,6-D-glucan binding, beta-1->6-D-glucan binding Sources: GOC:mengo_curators